{
  "gene_name": "Fibroblast growth factor receptor 4",
  "gene_symbol": "FGFR4",
  "term_label": "receptor complex",
  "gene": "UniProtKB:P22455",
  "term_id": "GO:0043235"
}